{
  "term_label": "mitochondrial electron transport, cytochrome c to oxygen",
  "gene_name": "Cytochrome c",
  "gene": "UniProtKB:P99999",
  "gene_symbol": "CYCS",
  "term_id": "GO:0006123"
}